acetylenedicarboxylate decarboxylase activity [GO:0050476] (molecular function) Relationships: is_a carboxy-lyase activity [GO:0016831] Also known as: acetylenedicarboxylate carboxy-lyase (pyruvate-forming), acetylenedicarboxylate carboxy-lyase activity, acetylenedicarboxylate hydrase activity, acetylenedicarboxylate hydratase activity Definition: Catalysis of the reaction: H2O + acetylenedicarboxylate = CO2 + pyruvate. Sources: EC:4.1.1.78